formimidoylglutamate deiminase activity [GO:0050416] (molecular function) Also known as: formiminoglutamate deiminase activity, N-formimidoyl-L-glutamate iminohydrolase activity, formiminoglutamic iminohydrolase activity Sources: EC:3.5.3.13, MetaCyc:FORMIMINOGLUTAMATE-DEIMINASE-RXN Relationships: is a type of GO:0016813 Definition: Catalysis of the reaction: N-formimidoyl-L-glutamate + H2O = N-formyl-L-glutamate + NH3.